epigenetic programming of gene expression [GO:0043045] (biological process) Definition: A epigenetic process that happens during embryonic development that modulates gene expression potential at later stages of development of the organism, including the adult. Epigenetic regulation takes place via chromatin remodeling either by modifying higher order chromatin fiber structure, nucleosomal histones, or cytosine DNA methylation. Relationships: is a type of epigenetic regulation of gene expression [GO:0040029] References: PMID:12138111, PMID:22868271 Sources: GOC:go_curators Also known as: DNA methylation involved in embryo development, de novo DNA methylation, epigenetic regulation of embryonic gene expression, post-fertilization epigenetic regulation of gene expression Subtypes: epigenetic programming in the zygotic pronuclei [GO:0044725], genomic imprinting [GO:0071514]